regulation of monoatomic anion transmembrane transport [GO:1903959] (biological process) Definition: Any process that modulates the frequency, rate or extent of anion transmembrane transport. Also known as: regulation of anion transmembrane transport Relationships: is a type of GO:0034765; is a type of regulation of monoatomic anion transport [GO:0044070]; regulates monoatomic anion transmembrane transport [GO:0098656] Sources: GOC:TermGenie, GOC:vw, GO_REF:0000058 Subtypes: GO:1903960, GO:1903961, regulation of iodide transmembrane transport [GO:1904212]